{
  "term_id": "GO:0005789",
  "term_label": "endoplasmic reticulum membrane",
  "gene_symbol": "PIGG",
  "gene_name": "GPI ethanolamine phosphate transferase 2",
  "gene": "UniProtKB:Q5H8A4"
}